{
  "gene_name": "Protein tyrosine phosphatase receptor type C-associated protein",
  "term_label": "Unknown biological process",
  "gene_symbol": "PTPRCAP",
  "term_id": "UNKNOWN:0002",
  "gene": "UniProtKB:Q14761"
}